{
  "gene_name": "Serine_threonine-protein kinase LMTK3",
  "gene_symbol": "LMTK3",
  "term_label": "Unknown cellular component",
  "term_id": "UNKNOWN:0003",
  "gene": "UniProtKB:Q96Q04"
}